{
  "term_label": "phosphatidylcholine metabolic process",
  "gene_symbol": "PLA2G2F",
  "gene": "UniProtKB:Q9BZM2",
  "term_id": "GO:0046470",
  "gene_name": "Group IIF secretory phospholipase A2"
}